{
  "gene_symbol": "IGLV3-19",
  "gene": "UniProtKB:P01714",
  "gene_name": "Immunoglobulin lambda variable 3-19",
  "term_id": "GO:0019814",
  "term_label": "immunoglobulin complex"
}